{
  "gene_symbol": "TONSL",
  "term_id": "GO:0043596",
  "gene": "UniProtKB:Q96HA7",
  "term_label": "nuclear replication fork",
  "gene_name": "Tonsoku-like protein"
}